{
  "term_id": "GO:0043005",
  "gene_symbol": "TPH1",
  "term_label": "neuron projection",
  "gene_name": "Tryptophan 5-hydroxylase 1",
  "gene": "UniProtKB:P17752"
}